negative regulation of ERBB signaling pathway [GO:1901185] (biological process) Also known as: down regulation of EGF receptor family signaling pathway, down regulation of ERBB signaling pathway, down regulation of ERBB signalling pathway, down regulation of ErbB signaling, down-regulation of EGF receptor family signaling pathway, down-regulation of ERBB signaling pathway, down-regulation of ERBB signalling pathway, down-regulation of ErbB signaling, downregulation of EGF receptor family signaling pathway, downregulation of ERBB signaling pathway, downregulation of ERBB signalling pathway, downregulation of ErbB signaling, inhibition of EGF receptor family signaling pathway, inhibition of ERBB signalling pathway, inhibition of ErbB signaling, negative regulation of EGF receptor family signaling pathway, negative regulation of ERBB signalling pathway, negative regulation of ErbB signaling, inhibition of ERBB signaling pathway, down regulation of EGFR family signaling pathway, down-regulation of EGFR family signaling pathway, downregulation of EGFR family signaling pathway, inhibition of EGFR family signaling pathway, negative regulation of EGFR family signaling pathway Sources: GOC:BHF, GOC:TermGenie Definition: Any process that stops, prevents or reduces the frequency, rate or extent of ERBB signaling pathway. Subtypes: negative regulation of epidermal growth factor receptor signaling pathway [GO:0042059], negative regulation of ERBB4 signaling pathway [GO:0120154], negative regulation of ERBB3 signaling pathway [GO:1905579] Relationships: is a type of negative regulation of signal transduction [GO:0009968]; is a type of regulation of ERBB signaling pathway [GO:1901184]; RO_0002212 ERBB signaling pathway [GO:0038127]